{
  "gene": "UniProtKB:Q92878",
  "term_id": "GO:0000722",
  "gene_symbol": "RAD50",
  "gene_name": "DNA repair protein RAD50",
  "term_label": "telomere maintenance via recombination"
}